{
  "gene": "UniProtKB:O60403",
  "gene_name": "Olfactory receptor 10H2",
  "gene_symbol": "OR10H2",
  "term_id": "GO:0004984",
  "term_label": "olfactory receptor activity"
}